7-methylguanosine mRNA capping [GO:0006370] (biological process) Definition: The sequence of enzymatic reactions by which the mRNA 5' cap structure, an inverted 7-methylguanosine linked via a 5'-5' triphosphate bridge (m7G(5')ppp(5')X) to the first transcribed residue, is added to a nascent transcript. Additional methylation can occur on the ribose sugars of the first and second nucleotides adjacent to the m7G nRNA cap. These methylations are often referred to as N6,2'-O-dimethyladenosine (m6,2A) and N6,2'-O-dimethylguanosine (m6,2G), respectively. References: PMID:9266685 Sources: GOC:mah Also known as: 5' end capping, 5'-end processing, 5' mRNA capping, 5'-end mRNA processing, mRNA capping Relationships: is a type of mRNA processing [GO:0006397]; is a type of 7-methylguanosine RNA capping [GO:0009452] Regulation: positively regulated by positive regulation of 7-methylguanosine mRNA capping [GO:0160199]